{
  "term_id": "UNKNOWN:0001",
  "gene_symbol": "ASZ1",
  "term_label": "Unknown molecular function",
  "gene_name": "Ankyrin repeat, SAM and basic leucine zipper domain-containing protein 1",
  "gene": "UniProtKB:Q8WWH4"
}